{
  "term_label": "membrane",
  "gene_name": "Aldehyde dehydrogenase, dimeric NADP-preferring",
  "term_id": "GO:0016020",
  "gene": "UniProtKB:P30838",
  "gene_symbol": "ALDH3A1"
}